{
  "term_label": "very long-chain fatty acid catabolic process",
  "gene": "UniProtKB:Q9UBJ2",
  "gene_name": "ATP-binding cassette sub-family D member 2",
  "gene_symbol": "ABCD2",
  "term_id": "GO:0042760"
}